{
  "gene_symbol": "CEP290",
  "term_label": "ciliary basal body-plasma membrane docking",
  "gene_name": "Centrosomal protein of 290 kDa",
  "gene": "UniProtKB:O15078",
  "term_id": "GO:0097711"
}